{
  "term_label": "Golgi organization",
  "term_id": "GO:0007030",
  "gene_symbol": "GOLGA8J",
  "gene": "UniProtKB:A6NMD2",
  "gene_name": "Golgin subfamily A member 8J"
}